embryonic hindlimb morphogenesis [GO:0035116] (biological process) Sources: ISBN:0198612001 Relationships: is a type of GO:0030326; is a type of hindlimb morphogenesis [GO:0035137] Definition: The process, occurring in the embryo, by which the anatomical structures of the hindlimbs are generated and organized. The hindlimbs are the posterior limbs of an animal.